{
  "gene": "UniProtKB:Q8NEV4",
  "gene_name": "Myosin-IIIa",
  "term_label": "microfilament motor activity",
  "gene_symbol": "MYO3A",
  "term_id": "GO:0000146"
}